{
  "term_label": "Unknown molecular function",
  "gene": "UniProtKB:Q8N999",
  "gene_name": "RNA ligase 1",
  "gene_symbol": "RLIG1",
  "term_id": "UNKNOWN:0001"
}